{
  "term_id": "GO:0005801",
  "term_label": "cis-Golgi network",
  "gene_name": "Golgin subfamily A member 8R",
  "gene_symbol": "GOLGA8R",
  "gene": "UniProtKB:I6L899"
}